cardiolipin metabolic process [GO:0032048] (biological process) Relationships: is a type of phosphatidylglycerol metabolic process [GO:0046471] Regulation: regulated by regulation of cardiolipin metabolic process [GO:1900208]; negatively regulated by negative regulation of cardiolipin metabolic process [GO:1900209]; positively regulated by positive regulation of cardiolipin metabolic process [GO:1900210] Also known as: cardiolipin metabolism, diphosphatidylglycerol metabolic process, diphosphatidylglycerol metabolism Sources: GOC:mah Definition: The chemical reactions and pathways involving cardiolipin, 1,3-bis(3-phosphatidyl)glycerol. Subtypes: cardiolipin biosynthetic process [GO:0032049], cardiolipin acyl-chain remodeling [GO:0035965]